{
  "term_id": "GO:0009897",
  "gene_symbol": "BTNL9",
  "gene_name": "Butyrophilin-like protein 9",
  "gene": "UniProtKB:Q6UXG8",
  "term_label": "external side of plasma membrane"
}